{
  "term_label": "fatty acyl-CoA hydrolase activity",
  "gene_name": "Peroxisomal succinyl-coenzyme A thioesterase",
  "gene": "UniProtKB:Q8N9L9",
  "term_id": "GO:0047617",
  "gene_symbol": "ACOT4"
}